{
  "gene_symbol": "ZNF346",
  "term_id": "UNKNOWN:0002",
  "gene_name": "Zinc finger protein 346",
  "gene": "UniProtKB:Q9UL40",
  "term_label": "Unknown biological process"
}